{
  "term_id": "GO:0045743",
  "gene_symbol": "DSTYK",
  "term_label": "positive regulation of fibroblast growth factor receptor signaling pathway",
  "gene_name": "Dual serine_threonine and tyrosine protein kinase",
  "gene": "UniProtKB:Q6XUX3"
}